regulation of cell adhesion involved in sprouting angiogenesis [GO:0106088] (biological process) Relationships: is a type of regulation of cell adhesion [GO:0030155]; regulates cell adhesion involved in sprouting angiogenesis [GO:0120078] Definition: Any process that modulates the frequency, rate or extent of cell adhesion involved in sprouting angiogenesis. References: PMID:24177325 Sources: GOC:BHF, GOC:BHF_miRNA, GOC:rph Subtypes: negative regulation of cell adhesion involved in sprouting angiogenesis [GO:0106089], positive regulation of cell adhesion involved in sprouting angiogenesis [GO:0106090]